{
  "gene_symbol": "STIP1",
  "gene": "UniProtKB:P31948",
  "term_id": "GO:0051879",
  "gene_name": "Stress-induced-phosphoprotein 1",
  "term_label": "Hsp90 protein binding"
}